{
  "term_id": "GO:0032012",
  "term_label": "regulation of ARF protein signal transduction",
  "gene_name": "ARF GTPase-activating protein GIT1",
  "gene_symbol": "GIT1",
  "gene": "UniProtKB:Q9Y2X7"
}